{
  "gene_name": "WD repeat-containing protein 44",
  "gene": "UniProtKB:Q5JSH3",
  "term_id": "GO:0010008",
  "term_label": "endosome membrane",
  "gene_symbol": "WDR44"
}